{
  "term_id": "GO:0005886",
  "gene_symbol": "HSP90AB4P",
  "gene": "UniProtKB:Q58FF6",
  "gene_name": "Putative heat shock protein HSP 90-beta 4",
  "term_label": "plasma membrane"
}